{
  "gene_symbol": "TSPEAR",
  "term_label": "signal transduction",
  "gene_name": "Thrombospondin-type laminin G domain and EAR repeat-containing protein",
  "term_id": "GO:0007165",
  "gene": "UniProtKB:Q8WU66"
}